{
  "gene": "UniProtKB:Q9H257",
  "term_label": "positive regulation of canonical NF-kappaB signal transduction",
  "term_id": "GO:0043123",
  "gene_name": "Caspase recruitment domain-containing protein 9",
  "gene_symbol": "CARD9"
}